cholestanetetraol 26-dehydrogenase activity [GO:0047748] (molecular function) Definition: Catalysis of the reaction: 5beta-cholestane-3alpha,7alpha,12alpha-triol + 5 H+ + 3 O2 + 6 reduced [adrenodoxin] = (25R)-3alpha,7alpha,12alpha-trihydroxy-5beta-cholestan-26-oate + 4 H2O + 6 oxidized [adrenodoxin]. Relationships: is a type of oxidoreductase activity, acting on paired donors, with incorporation or reduction of molecular oxygen, reduced iron-sulfur protein as one donor, and incorporation of one atom of oxygen [GO:0016713] Also known as: 5beta-cholestane-3alpha,7alpha,12alpha,26-tetraol:NAD+ 26-oxidoreductase activity, 5beta-cholestane-3alpha,7alpha,12alpha,26-tetrol dehydrogenase activity, TEHC-NAD oxidoreductase activity, cholestanetetrol 26-dehydrogenase activity Sources: RHEA:34631